{
  "term_label": "superoxide-generating NAD(P)H oxidase activity",
  "gene_symbol": "DUOX2",
  "gene": "UniProtKB:Q9NRD8",
  "term_id": "GO:0016175",
  "gene_name": "Dual oxidase 2"
}